{
  "gene_symbol": "ACER1",
  "gene": "UniProtKB:Q8TDN7",
  "term_id": "GO:0017040",
  "gene_name": "Alkaline ceramidase 1",
  "term_label": "N-acylsphingosine amidohydrolase activity"
}